{
  "term_id": "UNKNOWN:0003",
  "gene_symbol": "GFM2",
  "term_label": "Unknown cellular component",
  "gene": "UniProtKB:Q969S9",
  "gene_name": "Ribosome-releasing factor 2, mitochondrial"
}